{
  "gene": "UniProtKB:Q8NGI6",
  "term_label": "Unknown biological process",
  "gene_symbol": "OR4D10",
  "gene_name": "Olfactory receptor 4D10",
  "term_id": "UNKNOWN:0002"
}